{
  "gene_name": "Signal transducer CD24",
  "term_id": "GO:0030296",
  "term_label": "protein tyrosine kinase activator activity",
  "gene": "UniProtKB:P25063",
  "gene_symbol": "CD24"
}